{
  "gene_symbol": "IKZF2",
  "term_label": "RNA polymerase II cis-regulatory region sequence-specific DNA binding",
  "term_id": "GO:0000978",
  "gene": "UniProtKB:Q9UKS7",
  "gene_name": "Zinc finger protein Helios"
}